{
  "gene_symbol": "RXFP3",
  "gene": "UniProtKB:Q9NSD7",
  "term_label": "galanin receptor activity",
  "term_id": "GO:0004966",
  "gene_name": "Relaxin-3 receptor 1"
}